brexanolone biosynthetic process [GO:0062174] (BP) References: PMID:24390875 Relationships: is a type of steroid biosynthetic process [GO:0006694]; is a type of ketone biosynthetic process [GO:0042181]; is a type of brexanolone metabolic process [GO:0062173] Definition: The chemical reactions and pathways resulting in the formation of brexanolone. Also known as: allopregnanolone anabolism, allopregnanolone biosynthesis, allopregnanolone biosynthetic process, allopregnanolone synthesis, allotetrahydroprogesterone anabolism, allotetrahydroprogesterone biosynthesis, allotetrahydroprogesterone biosynthetic process, allotetrahydroprogesterone synthesis, brexanolone anabolism, brexanolone biosynthesis, brexanolone synthesis